{
  "gene_name": "Tyrosine-protein phosphatase non-receptor type 13",
  "term_label": "cytoplasm",
  "term_id": "GO:0005737",
  "gene_symbol": "PTPN13",
  "gene": "UniProtKB:Q12923"
}